{
  "gene_name": "Sorting nexin-30",
  "gene_symbol": "SNX30",
  "term_label": "endocytic recycling",
  "gene": "UniProtKB:Q5VWJ9",
  "term_id": "GO:0032456"
}